{
  "gene": "UniProtKB:Q8TD07",
  "gene_symbol": "RAET1E",
  "term_label": "external side of plasma membrane",
  "term_id": "GO:0009897",
  "gene_name": "Retinoic acid early transcript 1E"
}